{
  "gene_symbol": "TLCD3A",
  "gene": "UniProtKB:Q8TBR7",
  "term_id": "UNKNOWN:0001",
  "term_label": "Unknown molecular function",
  "gene_name": "TLC domain-containing protein 3A"
}